etioplast stroma [GO:0009578] (cellular component) Sources: GOC:jl Definition: The space enclosed by the double membrane of an etioplast but excluding the prothylakoid space. It contains the etioplast DNA. Relationships: is a type of GO:0009532; is part of GO:0009513